{
  "term_id": "GO:0018279",
  "gene_name": "Dolichyl-diphosphooligosaccharide--protein glycosyltransferase subunit 1",
  "gene": "UniProtKB:P04843",
  "gene_symbol": "RPN1",
  "term_label": "protein N-linked glycosylation via asparagine"
}